{
  "gene": "UniProtKB:Q8WWL2",
  "term_label": "cytoplasmic vesicle membrane",
  "gene_name": "Protein spire homolog 2",
  "gene_symbol": "SPIRE2",
  "term_id": "GO:0030659"
}